positive regulation of cold-induced thermogenesis [GO:0120162] (biological process) References: PMID:27876809 Also known as: positive regulation of CIT Definition: Any process that activates or increases the frequency, rate or extent of cold-induced thermogenesis. Relationships: is a type of positive regulation of metabolic process [GO:0009893]; is a type of positive regulation of multicellular organismal process [GO:0051240]; is a type of regulation of cold-induced thermogenesis [GO:0120161]; positively regulates cold-induced thermogenesis [GO:0106106]